laminin-1 binding [GO:0043237] (molecular function) Relationships: is a type of laminin binding [GO:0043236] Definition: Binding to laminin-1, a glycoprotein trimer with the subunit composition alpha1, beta1, gamma1. Also known as: laminin-111 binding Sources: GOC:go_curators